{
  "term_label": "plasma membrane",
  "gene_symbol": "SYT15B",
  "gene": "UniProtKB:X6R8R1",
  "gene_name": "Synaptotagmin-15B",
  "term_id": "GO:0005886"
}